methionine transport [GO:0015821] (BP) Relationships: is a type of GO:0000101; is a type of amino acid transport [GO:0006865]; is a type of organic cation transport [GO:0015695] Subtypes: D-methionine transmembrane transport [GO:0048473], GO:1903692 Also known as: L-methionine transport Sources: GOC:ai Definition: The directed movement of methionine, 2-amino-4-(methylthio)butanoic acid, into, out of or within a cell, or between cells, by means of some agent such as a transporter or pore.